{
  "gene_name": "X antigen family member 5",
  "term_label": "Unknown biological process",
  "term_id": "UNKNOWN:0002",
  "gene_symbol": "XAGE5",
  "gene": "UniProtKB:Q8WWM1"
}